{
  "gene_name": "P antigen family member 1",
  "gene_symbol": "PAGE1",
  "term_label": "Unknown cellular component",
  "term_id": "UNKNOWN:0003",
  "gene": "UniProtKB:O75459"
}